{
  "term_label": "Unknown molecular function",
  "gene_symbol": "PIH1D2",
  "term_id": "UNKNOWN:0001",
  "gene_name": "PIH1 domain-containing protein 2",
  "gene": "UniProtKB:Q8WWB5"
}